{
  "gene": "UniProtKB:P79483",
  "term_id": "GO:0031902",
  "gene_symbol": "HLA-DRB3",
  "term_label": "late endosome membrane",
  "gene_name": "HLA class II histocompatibility antigen, DR beta 3 chain"
}